{
  "gene_symbol": "GABRG1",
  "gene": "UniProtKB:Q8N1C3",
  "term_label": "gamma-aminobutyric acid signaling pathway",
  "gene_name": "Gamma-aminobutyric acid receptor subunit gamma-1",
  "term_id": "GO:0007214"
}